negative regulation of protein import into nucleus during spindle assembly checkpoint [GO:1901925] (biological process) References: PMID:23177738 Sources: GOC:TermGenie, GOC:dgf Also known as: negative regulation of protein import into nucleus during mitotic cell cycle spindle assembly checkpoint, KTIP, Kap121p transport inhibitory pathway Definition: Any process that stops, prevents, or reduces the frequency, rate or extent of the movement of proteins from the cytoplasm into the nucleus, and that occurs as a response to the mitotic cell cycle spindle assembly checkpoint. In S. cerevisiae, this process involves inhibition of the karyopherin/importin Kap121p (also known as Pse1p), which acts as the specific nuclear import receptor for several proteins, including Glc7p. Glc7p functions in opposition to key spindle assembly checkpoint protein Aurora kinase (Ipl1p). Relationships: is a type of GO:0072479